{
  "gene_symbol": "CDON",
  "term_label": "nervous system development",
  "gene": "UniProtKB:Q4KMG0",
  "term_id": "GO:0007399",
  "gene_name": "Cell adhesion molecule-related_down-regulated by oncogenes"
}